{
  "term_id": "GO:0030424",
  "gene_symbol": "VSTM5",
  "term_label": "axon",
  "gene": "UniProtKB:A8MXK1",
  "gene_name": "V-set and transmembrane domain-containing protein 5"
}